{
  "term_label": "Unknown biological process",
  "gene": "UniProtKB:O75711",
  "gene_symbol": "SCRG1",
  "gene_name": "Scrapie-responsive protein 1",
  "term_id": "UNKNOWN:0002"
}